{
  "term_id": "GO:0051260",
  "gene_name": "RING finger protein 112",
  "gene_symbol": "RNF112",
  "gene": "UniProtKB:Q9ULX5",
  "term_label": "protein homooligomerization"
}